{
  "gene_symbol": "GCM2",
  "gene": "UniProtKB:O75603",
  "term_id": "GO:0005634",
  "gene_name": "Chorion-specific transcription factor GCMb",
  "term_label": "nucleus"
}